{
  "gene_symbol": "FOXA2",
  "gene": "UniProtKB:Q9Y261",
  "term_id": "GO:0030154",
  "gene_name": "Hepatocyte nuclear factor 3-beta",
  "term_label": "cell differentiation"
}